positive regulation of transdifferentiation [GO:1903620] (biological process) Definition: Any process that activates or increases the frequency, rate or extent of transdifferentiation. References: PMID:22118091 Sources: GOC:TermGenie, GO_REF:0000058 Also known as: up regulation of transdifferentiation, up-regulation of transdifferentiation, upregulation of transdifferentiation, activation of transdifferentiation Relationships: is a type of GO:0045597; is a type of regulation of transdifferentiation [GO:1903618]; positively regulates GO:0060290